{
  "gene_symbol": "MINDY3",
  "term_id": "GO:1990380",
  "gene": "UniProtKB:Q9H8M7",
  "term_label": "K48-linked deubiquitinase activity",
  "gene_name": "Ubiquitin carboxyl-terminal hydrolase MINDY-3"
}